{
  "term_label": "regulation of actin cytoskeleton organization",
  "gene": "UniProtKB:O94844",
  "gene_name": "Rho-related BTB domain-containing protein 1",
  "term_id": "GO:0032956",
  "gene_symbol": "RHOBTB1"
}